{
  "term_label": "acid phosphatase activity",
  "gene_symbol": "MDP1",
  "gene": "UniProtKB:Q86V88",
  "gene_name": "Magnesium-dependent phosphatase 1",
  "term_id": "GO:0003993"
}